lactate dehydrogenase activity [GO:0004457] (molecular function) Definition: Catalysis of the reaction: lactate + NAD+ = H+ + NADH + pyruvate. Sources: GOC:ai, GOC:bf Relationships: is a type of oxidoreductase activity, acting on CH-OH group of donors [GO:0016614] Subtypes: GO:0047809, GO:0140171